{
  "gene_name": "G-protein coupled receptor 37-like 1",
  "gene_symbol": "GPR37L1",
  "gene": "UniProtKB:O60883",
  "term_id": "GO:0043235",
  "term_label": "receptor complex"
}